{
  "gene": "UniProtKB:Q9NTJ4",
  "gene_name": "Alpha-mannosidase 2C1",
  "gene_symbol": "MAN2C1",
  "term_label": "oligosaccharide catabolic process",
  "term_id": "GO:0009313"
}